{
  "term_label": "histone H3K9 demethylase activity",
  "term_id": "GO:0032454",
  "gene": "UniProtKB:Q15652",
  "gene_name": "Probable JmjC domain-containing histone demethylation protein 2C",
  "gene_symbol": "JMJD1C"
}